{
  "gene_symbol": "PKD1L1",
  "gene": "UniProtKB:Q8TDX9",
  "term_label": "membrane",
  "term_id": "GO:0016020",
  "gene_name": "Polycystin-1-like protein 1"
}